regulation of apoptotic process involved in outflow tract morphogenesis [GO:1902256] (biological process) Also known as: regulation of apoptosis involved in outflow tract morphogenesis Relationships: is a type of regulation of apoptotic process involved in morphogenesis [GO:1902337]; regulates apoptotic process involved in outflow tract morphogenesis [GO:0003275] Definition: Any process that modulates the frequency, rate or extent of apoptotic process involved in outflow tract morphogenesis. References: PMID:16839542 Sources: GOC:TermGenie, GOC:dph, GOC:mtg_apoptosis Subtypes: negative regulation of apoptotic process involved in outflow tract morphogenesis [GO:1902257], positive regulation of apoptotic process involved in outflow tract morphogenesis [GO:1902258]